{
  "gene": "UniProtKB:Q147X3",
  "gene_name": "N-alpha-acetyltransferase 30",
  "term_label": "Unknown biological process",
  "gene_symbol": "NAA30",
  "term_id": "UNKNOWN:0002"
}